{
  "term_label": "nucleus",
  "term_id": "GO:0005634",
  "gene_name": "Poly(rC)-binding protein 3",
  "gene_symbol": "PCBP3",
  "gene": "UniProtKB:P57721"
}